{
  "term_id": "UNKNOWN:0002",
  "gene": "UniProtKB:A0A1B0GVY2",
  "term_label": "Unknown biological process",
  "gene_symbol": "LOC122455340",
  "gene_name": "Uncharacterized protein"
}